response to progesterone [GO:0032570] (biological process) Also known as: response to progesterone stimulus Sources: GOC:sl Relationships: is a type of response to steroid hormone [GO:0048545]; is a type of GO:1901654 Subtypes: GO:0071393 Definition: Any process that results in a change in state or activity of a cell or an organism (in terms of movement, secretion, enzyme production, gene expression, etc.) as a result of a progesterone stimulus.